{
  "gene": "UniProtKB:Q6VY07",
  "gene_name": "Phosphofurin acidic cluster sorting protein 1",
  "gene_symbol": "PACS1",
  "term_label": "protein localization to plasma membrane",
  "term_id": "GO:0072659"
}